5'-adenylyl sulfate transmembrane transport [GO:1902558] (biological process) References: PMID:24296033 Sources: GOC:TermGenie Subtypes: mitochondrial 5'-adenylyl sulfate transmembrane transport [GO:1990553] Definition: The process in which 5'-adenylyl sulfate is transported across a membrane. Relationships: is a type of organic anion transport [GO:0015711]; is a type of purine ribonucleotide transport [GO:0015868]; is a type of GO:0051503; is a type of GO:0072348; is a type of purine-containing compound transmembrane transport [GO:0072530]; is a type of nucleotide transmembrane transport [GO:1901679] Also known as: adenosine 5'-phosphosulfate transmembrane transport